{
  "gene_symbol": "ATG2B",
  "term_label": "pexophagy",
  "gene_name": "Autophagy-related protein 2 homolog B",
  "term_id": "GO:0000425",
  "gene": "UniProtKB:Q96BY7"
}